regulation of the force of heart contraction by chemical signal [GO:0003057] (biological process) Also known as: chemical cardiac inotropy, regulation of the force of heart muscle contraction by chemical signal Sources: GOC:mtg_cardio, GOC:rl Subtypes: hormonal regulation of the force of heart contraction [GO:0003058], positive regulation of the force of heart contraction by chemical signal [GO:0003099], negative regulation of the force of heart contraction by chemical signal [GO:0003108] Definition: The regulation of the force of heart muscle contraction mediated by chemical signaling, hormonal, autocrine or paracrine. Relationships: is a type of GO:0002026